regulation of intermediate filament polymerization [GO:0030839] (biological process) Sources: GOC:mah Definition: Any process that modulates the frequency, rate or extent of the assembly of intermediate filaments by the addition of monomers to a filament. Subtypes: negative regulation of intermediate filament polymerization [GO:0030840], positive regulation of intermediate filament polymerization [GO:0030841] Relationships: is a type of regulation of protein polymerization [GO:0032271]; is a type of regulation of intermediate filament polymerization or depolymerization [GO:0045108]; regulates intermediate filament polymerization [GO:0045107]